ATP-dependent citrate lyase complex [GO:0140615] (CC) Also known as: citrate lyase complex, citrate synthase complex Definition: A protein complex that catalyzes the cleavage of citrate into oxaloacetate and acetyl-CoA. References: PMID:12376641 Relationships: is a type of transferase complex [GO:1990234]